 [rdf-schema#label]